{
  "gene": "UniProtKB:Q9P2W7",
  "gene_symbol": "B3GAT1",
  "term_id": "GO:0005975",
  "gene_name": "Galactosylgalactosylxylosylprotein 3-beta-glucuronosyltransferase 1",
  "term_label": "carbohydrate metabolic process"
}